{
  "term_id": "GO:0050766",
  "term_label": "positive regulation of phagocytosis",
  "gene_symbol": "FCGR2B",
  "gene_name": "Low affinity immunoglobulin gamma Fc region receptor II-b",
  "gene": "UniProtKB:P31994"
}